{
  "gene": "UniProtKB:Q13315",
  "term_label": "DNA damage checkpoint signaling",
  "gene_name": "Serine-protein kinase ATM",
  "gene_symbol": "ATM",
  "term_id": "GO:0000077"
}